regulation of maternal process involved in parturition [GO:1904301] (biological process) Definition: Any process that modulates the frequency, rate or extent of maternal process involved in parturition. References: PMID:1849751 Sources: GOC:TermGenie, GO_REF:0000058 Relationships: is a type of regulation of multicellular organismal process [GO:0051239]; is a type of regulation of reproductive process [GO:2000241]; RO_0002211 GO:0060137 Subtypes: negative regulation of maternal process involved in parturition [GO:1904302], positive regulation of maternal process involved in parturition [GO:1904303]